response to protozoan [GO:0001562] (biological process) Also known as: response to protozoa, response to protozoon, resistance to pathogenic protozoa Sources: GOC:ai Subtypes: GO:0001563, defense response to protozoan [GO:0042832], cellular response to protozoan [GO:0099141] Definition: Any process that results in a change in state or activity of a cell or an organism (in terms of movement, secretion, enzyme production, gene expression, etc.) as a result of a stimulus from a protozoan. Relationships: is a type of GO:0051707